megasome [GO:0043246] (cellular component) References: PMID:11206117, PMID:1999020 Relationships: is a type of lysosome [GO:0005764] Definition: Large, cysteine proteinase rich lysosomes, often found in the amastigote (an intracytoplasmic, nonflagellated form of the parasite) stage of Leishmania species belonging to the mexicana complex.